{
  "term_id": "UNKNOWN:0001",
  "gene_name": "Semenogelin-2",
  "gene_symbol": "SEMG2",
  "gene": "UniProtKB:Q02383",
  "term_label": "Unknown molecular function"
}